maintenance of seed dormancy by absisic acid [GO:0098755] (biological process) Relationships: is_a maintenance of seed dormancy [GO:0010231]; is part of GO:0009737 Definition: The process by which seed dormancy is maintained by the presence of absisic acid. References: PMID:9580097 Sources: GOC:dos